{
  "term_id": "GO:0000472",
  "gene_name": "Transducin beta-like protein 3",
  "gene_symbol": "TBL3",
  "gene": "UniProtKB:Q12788",
  "term_label": "endonucleolytic cleavage to generate mature 5'-end of SSU-rRNA from (SSU-rRNA, 5.8S rRNA, LSU-rRNA)"
}